{
  "term_label": "Unknown molecular function",
  "gene_name": "Zinc finger protein 618",
  "term_id": "UNKNOWN:0001",
  "gene": "UniProtKB:Q5T7W0",
  "gene_symbol": "ZNF618"
}